{
  "term_id": "GO:0099634",
  "gene": "UniProtKB:Q8N0W4",
  "term_label": "postsynaptic specialization membrane",
  "gene_name": "Neuroligin-4, X-linked",
  "gene_symbol": "NLGN4X"
}